regulation of oligopeptide transport [GO:0090088] (biological process) Definition: Any process that modulates the frequency, rate or extent of the directed movement of oligopeptides into, out of or within a cell, or between cells, by means of some agent such as a transporter or pore. Oligopeptides are molecules that contain a small number (2 to 20) of amino-acid residues connected by peptide linkages. Sources: GOC:dph, GOC:tb Subtypes: GO:0090089, negative regulation of oligopeptide transport [GO:2000877], GO:2000878 Relationships: is a type of regulation of peptide transport [GO:0090087]; RO_0002211 oligopeptide transport [GO:0006857]